{
  "gene_symbol": "SIDT2",
  "gene_name": "SID1 transmembrane family member 2",
  "term_label": "double-stranded RNA binding",
  "term_id": "GO:0003725",
  "gene": "UniProtKB:Q8NBJ9"
}